{
  "term_id": "GO:0005886",
  "term_label": "plasma membrane",
  "gene_name": "Probable G-protein coupled receptor 173",
  "gene_symbol": "GPR173",
  "gene": "UniProtKB:Q9NS66"
}